aerobic respiration [GO:0009060] (biological process) Relationships: is a type of GO:0045333 Subtypes: GO:0006119, alternative respiration [GO:0010230], aerobic respiration, using nitrite as electron donor [GO:0019332], aerobic respiration, using ammonia as electron donor [GO:0019409], GO:0019410, aerobic respiration, using ferrous ions as electron donor [GO:0019411], aerobic respiration, using hydrogen as electron donor [GO:0019412], aerobic respiration, using sulfur or sulfate as electron donor [GO:0019414], aerobic electron transport chain [GO:0019646], GO:0043554 Sources: GOC:das, GOC:jl, ISBN:0140513590 Definition: The enzymatic release of energy from inorganic and organic compounds (especially carbohydrates and fats) which requires oxygen as the terminal electron acceptor. Regulation: regulated by regulation of aerobic respiration [GO:1903715]